aromatic-amino-acid-glyoxylate transaminase activity [GO:0047313] (molecular function) Definition: Catalysis of the reaction: glyoxylate + an aromatic amino acid = L-glycine + an aromatic oxo acid. Also known as: aromatic-amino-acid-glyoxylate aminotransferase activity, aromatic-amino-acid--glyoxylate aminotransferase activity, aromatic-amino-acid:glyoxylate aminotransferase activity Sources: EC:2.6.1.60, MetaCyc:2.6.1.60-RXN Relationships: is a type of transaminase activity [GO:0008483]